{
  "gene_name": "Protein unc-119 homolog A",
  "term_id": "GO:0051233",
  "gene": "UniProtKB:Q13432",
  "term_label": "spindle midzone",
  "gene_symbol": "UNC119"
}